cytosolic proteasome regulatory particle [GO:0031600] (cellular component) Sources: GOC:mah, GOC:mtg_sensu Relationships: is a type of proteasome regulatory particle [GO:0005838]; is part of cytosolic proteasome complex [GO:0031597] Definition: A multisubunit complex located in the cytosol of a cell, which caps one or both ends of the proteasome core complex. This complex recognizes, unfolds ubiquitinated proteins and translocates them to the proteasome core complex.